{
  "gene_symbol": "IGHV3-30-3",
  "gene": "UniProtKB:P0DP02",
  "gene_name": "Immunoglobulin heavy variable 3-30-3",
  "term_id": "GO:0003823",
  "term_label": "antigen binding"
}